3'-phosphoadenosine 5'-phosphosulfate biosynthetic process [GO:0050428] (biological process) Relationships: is_a purine ribonucleotide biosynthetic process [GO:0009152]; is a type of GO:0034036; is a type of sulfur compound biosynthetic process [GO:0044272]; is a type of 3'-phosphoadenosine 5'-phosphosulfate metabolic process [GO:0050427] Sources: ISBN:0198506732 Also known as: 3'-phosphoadenosine 5'-phosphosulfate anabolism, 3'-phosphoadenosine 5'-phosphosulfate biosynthesis, 3'-phosphoadenosine 5'-phosphosulfate formation, 3'-phosphoadenosine 5'-phosphosulfate synthesis, 3'-phosphoadenosine 5'-phosphosulphate biosynthesis, 3'-phosphoadenosine 5'-phosphosulphate biosynthetic process, 3'-phosphoadenylyl-sulfate biosynthesis, 3'-phosphoadenylyl-sulfate biosynthetic process, PAPS biosynthesis, PAPS biosynthetic process, adenosine 3'-phosphate 5'-phosphosulfate biosynthesis, adenosine 3'-phosphate 5'-phosphosulfate biosynthetic process, phosphoadenosine phosphosulfate biosynthesis, phosphoadenosine phosphosulfate biosynthetic process Definition: The chemical reactions and pathways resulting in the formation of 3'-phosphoadenosine 5'-phosphosulfate, a naturally occurring mixed anhydride. It is an intermediate in the formation of a variety of sulfo compounds in biological systems.